{
  "gene_symbol": "TMEM131L",
  "gene": "UniProtKB:A2VDJ0",
  "term_label": "Unknown molecular function",
  "gene_name": "Transmembrane protein 131-like",
  "term_id": "UNKNOWN:0001"
}